{
  "gene_symbol": "ZFR",
  "term_id": "UNKNOWN:0002",
  "gene_name": "Zinc finger RNA-binding protein",
  "term_label": "Unknown biological process",
  "gene": "UniProtKB:Q96KR1"
}